{
  "gene": "UniProtKB:Q9NS40",
  "gene_name": "Potassium voltage-gated channel subfamily H member 7",
  "gene_symbol": "KCNH7",
  "term_id": "GO:0005886",
  "term_label": "plasma membrane"
}